regulation of secretory granule organization [GO:1904409] (biological process) Subtypes: negative regulation of secretory granule organization [GO:1904410], positive regulation of secretory granule organization [GO:1904411] Definition: Any process that modulates the frequency, rate or extent of secretory granule organization. Also known as: regulation of secretory granule organisation, regulation of secretory granule organization and biogenesis References: PMID:15039777 Sources: GOC:TermGenie, GO_REF:0000058 Relationships: is a type of regulation of organelle organization [GO:0033043]; regulates secretory granule organization [GO:0033363]